{
  "gene": "UniProtKB:Q9H3J6",
  "term_label": "Unknown molecular function",
  "gene_symbol": "MTRFR",
  "gene_name": "Mitochondrial translation release factor in rescue",
  "term_id": "UNKNOWN:0001"
}